{
  "term_label": "follicle-stimulating hormone signaling pathway",
  "gene_symbol": "FSHB",
  "gene_name": "Follitropin subunit beta",
  "gene": "UniProtKB:P01225",
  "term_id": "GO:0042699"
}